positive regulation of telomere maintenance via telomere lengthening [GO:1904358] (biological process) Definition: Any process that activates or increases the frequency, rate or extent of telomere maintenance via telomere lengthening. Also known as: up regulation of telomere maintenance via telomere lengthening, up-regulation of telomere maintenance via telomere lengthening, upregulation of telomere maintenance via telomere lengthening, activation of telomere maintenance via telomere lengthening Relationships: is_a positive regulation of telomere maintenance [GO:0032206]; is a type of GO:1904356; positively regulates telomere maintenance via telomere lengthening [GO:0010833] References: PMID:23959892 Sources: GOC:BHF, GOC:BHF_telomere, GOC:TermGenie, GOC:nc, GO_REF:0000058 Subtypes: positive regulation of telomere maintenance via telomerase [GO:0032212]